regulation of (Z)-nonadeca-1,14-diene biosynthetic process [GO:1900941] (biological process) Subtypes: negative regulation of (Z)-nonadeca-1,14-diene biosynthetic process [GO:1900942], GO:1900943 Sources: GOC:TermGenie, GOC:mengo_curators Definition: Any process that modulates the frequency, rate or extent of (Z)-nonadeca-1,14-diene biosynthetic process. Also known as: regulation of (Z)-nonadeca-1,14-diene anabolism, regulation of (Z)-nonadeca-1,14-diene biosynthesis, regulation of (Z)-nonadeca-1,14-diene formation, regulation of (Z)-nonadeca-1,14-diene synthesis Relationships: is a type of regulation of olefin biosynthetic process [GO:1900911]; regulates (Z)-nonadeca-1,14-diene biosynthetic process [GO:1900879]